{
  "gene_symbol": "CTNNAL1",
  "term_label": "Unknown cellular component",
  "gene_name": "Alpha-catulin",
  "term_id": "UNKNOWN:0003",
  "gene": "UniProtKB:Q9UBT7"
}